{
  "gene_name": "Pre-mRNA-splicing factor 38A",
  "gene": "UniProtKB:Q8NAV1",
  "gene_symbol": "PRPF38A",
  "term_label": "precatalytic spliceosome",
  "term_id": "GO:0071011"
}